{
  "term_label": "Unknown cellular component",
  "term_id": "UNKNOWN:0003",
  "gene_symbol": "ATP5PD",
  "gene_name": "ATP synthase subunit d, mitochondrial",
  "gene": "UniProtKB:O75947"
}